heme export from vacuole to cytoplasm [GO:0140357] (biological process) References: PMID:28193844 Relationships: is a type of GO:0034486; is a type of heme transmembrane transport [GO:0035351] Definition: The directed movement of heme from inside the vacuole across the vacuolar membrane and into the cytosol.